L-serine conjugated cholate hydrolase activity [GO:7770004] (molecular function) Definition: Catalysis of the reaction: cholate + L-serine = L-serocholate + H2O. Relationships: is a type of amino acid conjugated cholate hydrolase activity [GO:7770003] References: PMID:38326609 Sources: RHEA:79139